{
  "gene_name": "Ubiquitin thioesterase OTUB2",
  "gene": "UniProtKB:Q96DC9",
  "term_label": "Unknown cellular component",
  "gene_symbol": "OTUB2",
  "term_id": "UNKNOWN:0003"
}